nuclear dicing body assembly [GO:1904258] (biological process) Relationships: is a type of GO:0030575; is a type of membraneless organelle assembly [GO:0140694] Definition: The aggregation, arrangement and bonding together of a set of components to form a nuclear dicing body. Also known as: D body assembly, D body formation, nuclear dicing body formation References: PMID:25902521 Sources: GOC:TermGenie, GO_REF:0000079